{
  "gene_symbol": "LAMA4",
  "term_label": "basement membrane",
  "term_id": "GO:0005604",
  "gene": "UniProtKB:Q16363",
  "gene_name": "Laminin subunit alpha-4"
}